glycerol-1,2-cyclic-phosphate 2-phosphodiesterase activity [GO:0047393] (molecular function) Also known as: rac-glycerol 1:2-cyclic phosphate 2-phosphodiesterase activity, rac-glycerol-1,2-cyclic-phosphate 2-glycerophosphohydrolase activity Definition: Catalysis of the reaction: glycerol 1,2-cyclic phosphate + H2O = glycerol 1-phosphate + H+. Sources: EC:3.1.4.42, RHEA:16493 Relationships: is a type of phosphoric diester hydrolase activity [GO:0008081]